{
  "gene_symbol": "GPALPP1",
  "gene": "UniProtKB:Q8IXQ4",
  "term_label": "Unknown molecular function",
  "gene_name": "GPALPP motifs-containing protein 1",
  "term_id": "UNKNOWN:0001"
}